{
  "gene_symbol": "WSCD1",
  "gene_name": "Sialate:O-sulfotransferase 1",
  "term_label": "Unknown biological process",
  "term_id": "UNKNOWN:0002",
  "gene": "UniProtKB:Q658N2"
}